lymph node development [GO:0048535] (biological process) Sources: GOC:add, ISBN:068340007X, ISBN:0781735149 Relationships: is a type of hematopoietic or lymphoid organ development [GO:0048534] Definition: The process whose specific outcome is the progression of lymph nodes over time, from their formation to the mature structure. A lymph node is a round, oval, or bean shaped structure localized in clusters along the lymphatic vessels, with a distinct internal structure including specialized vasculature and B- and T-zones for the activation of lymphocytes. Also known as: lymph gland development